{
  "gene_name": "Protein transport protein Sec24C",
  "gene_symbol": "SEC24C",
  "term_id": "GO:0030127",
  "gene": "UniProtKB:P53992",
  "term_label": "COPII vesicle coat"
}